{
  "gene_name": "Homocysteine-responsive endoplasmic reticulum-resident ubiquitin-like domain member 1 protein",
  "gene_symbol": "HERPUD1",
  "term_label": "negative regulation of endoplasmic reticulum stress-induced intrinsic apoptotic signaling pathway",
  "gene": "UniProtKB:Q15011",
  "term_id": "GO:1902236"
}